{
  "term_label": "L-glutamate transmembrane transport",
  "term_id": "GO:0015813",
  "gene_name": "Neutral amino acid transporter A",
  "gene": "UniProtKB:P43007",
  "gene_symbol": "SLC1A4"
}